{
  "gene_name": "Substance-P receptor",
  "term_id": "GO:1902093",
  "gene_symbol": "TACR1",
  "gene": "UniProtKB:P25103",
  "term_label": "positive regulation of flagellated sperm motility"
}